{
  "term_label": "intracellular signal transduction",
  "term_id": "GO:0035556",
  "gene_symbol": "SH3BP5",
  "gene_name": "SH3 domain-binding protein 5",
  "gene": "UniProtKB:O60239"
}